{
  "gene_symbol": "EBNA1BP2",
  "gene": "UniProtKB:Q99848",
  "term_id": "GO:0030687",
  "term_label": "preribosome, large subunit precursor",
  "gene_name": "Probable rRNA-processing protein EBP2"
}